{
  "term_label": "transcription factor TFTC complex",
  "gene_symbol": "TAF9",
  "term_id": "GO:0033276",
  "gene_name": "Transcription initiation factor TFIID subunit 9",
  "gene": "UniProtKB:Q16594"
}